{
  "gene_name": "Olfactory receptor 8J1",
  "gene": "UniProtKB:Q8NGP2",
  "term_id": "UNKNOWN:0003",
  "term_label": "Unknown cellular component",
  "gene_symbol": "OR8J1"
}